{
  "gene_name": "Protein shisa-9",
  "gene_symbol": "SHISA9",
  "gene": "UniProtKB:B4DS77",
  "term_label": "postsynaptic density",
  "term_id": "GO:0014069"
}